{
  "gene": "UniProtKB:P06730",
  "gene_symbol": "EIF4E",
  "gene_name": "Eukaryotic translation initiation factor 4E",
  "term_label": "translation initiation factor activity",
  "term_id": "GO:0003743"
}